{
  "gene": "UniProtKB:Q96ID5",
  "term_label": "Unknown molecular function",
  "term_id": "UNKNOWN:0001",
  "gene_symbol": "IGSF21",
  "gene_name": "Immunoglobulin superfamily member 21"
}